{
  "gene_name": "Uncharacterized protein KIAA0408",
  "gene": "UniProtKB:Q6ZU52",
  "gene_symbol": "KIAA0408",
  "term_id": "UNKNOWN:0002",
  "term_label": "Unknown biological process"
}